{
  "gene_symbol": "KEL",
  "gene_name": "Kell blood group glycoprotein",
  "gene": "UniProtKB:P23276",
  "term_id": "GO:0004222",
  "term_label": "metalloendopeptidase activity"
}